{
  "term_label": "Unknown biological process",
  "gene_symbol": "BPGM",
  "gene": "UniProtKB:P07738",
  "gene_name": "Bisphosphoglycerate mutase",
  "term_id": "UNKNOWN:0002"
}